{
  "gene_name": "Dynein axonemal heavy chain 9",
  "gene_symbol": "DNAH9",
  "term_id": "GO:0005930",
  "gene": "UniProtKB:Q9NYC9",
  "term_label": "axoneme"
}